eclosion [GO:0007562] (biological process) Definition: The emergence of an adult insect from a pupa case. Sources: GOC:dgh, GOC:dos, GOC:mah, ISBN:0198600461 Relationships: is a type of organism emergence from protective structure [GO:0071684]; is part of multicellular organism development [GO:0007275] Regulation: regulated by regulation of eclosion [GO:0007563]; negatively regulated by negative regulation of eclosion [GO:0045804]; positively regulated by positive regulation of eclosion [GO:0045805]